P-type manganese transporter activity [GO:0140613] (molecular function) Definition: Enables the transfer of a solute or solutes from one side of a membrane to the other according to the reaction: ATP + H2O + Mn2+(in) = ADP + H+ + Mn2+(out) + phosphate. References: PMID:11134055, PMID:15590060, PMID:15831496, PMID:21187401 Sources: RHEA:66820 Relationships: is a type of manganese ion transmembrane transporter activity [GO:0005384]; is a type of P-type ion transporter activity [GO:0015662]; is a type of ATPase-coupled monoatomic cation transmembrane transporter activity [GO:0019829]